{
  "gene_symbol": "CCL4L1",
  "gene": "UniProtKB:Q8NHW4",
  "term_id": "GO:0048245",
  "gene_name": "C-C motif chemokine 4-like",
  "term_label": "eosinophil chemotaxis"
}